{
  "term_id": "GO:0016192",
  "term_label": "vesicle-mediated transport",
  "gene_symbol": "RAB36",
  "gene": "UniProtKB:O95755",
  "gene_name": "Ras-related protein Rab-36"
}